{
  "term_id": "GO:0008251",
  "gene_name": "Adenosine deaminase domain-containing protein 1",
  "term_label": "tRNA-specific adenosine deaminase activity",
  "gene": "UniProtKB:Q96M93",
  "gene_symbol": "ADAD1"
}